{
  "term_label": "olfactory receptor activity",
  "term_id": "GO:0004984",
  "gene_symbol": "OR13A1",
  "gene": "UniProtKB:Q8NGR1",
  "gene_name": "Olfactory receptor 13A1"
}